{
  "gene": "UniProtKB:O60896",
  "gene_symbol": "RAMP3",
  "term_id": "GO:0072659",
  "gene_name": "Receptor activity-modifying protein 3",
  "term_label": "protein localization to plasma membrane"
}